negative regulation of tRNA processing [GO:2000236] (biological process) Sources: GOC:mah Also known as: negative regulation of tRNA maturation Relationships: is_a negative regulation of gene expression [GO:0010629]; is a type of negative regulation of tRNA metabolic process [GO:1903327]; is a type of GO:2000235; negatively regulates tRNA processing [GO:0008033] Definition: Any process that stops, prevents, or reduces the frequency, rate or extent of tRNA processing.